{
  "gene_symbol": "GATAD1",
  "gene": "UniProtKB:Q8WUU5",
  "term_label": "nucleus",
  "term_id": "GO:0005634",
  "gene_name": "GATA zinc finger domain-containing protein 1"
}